{
  "gene_name": "Ras-related C3 botulinum toxin substrate 2",
  "term_id": "GO:0030865",
  "gene_symbol": "RAC2",
  "term_label": "cortical cytoskeleton organization",
  "gene": "UniProtKB:P15153"
}